{
  "term_label": "protein localization involved in establishment of planar polarity",
  "term_id": "GO:0090251",
  "gene": "UniProtKB:O15259",
  "gene_name": "Nephrocystin-1",
  "gene_symbol": "NPHP1"
}